{
  "term_label": "N-terminal protein N-methyltransferase activity",
  "gene_symbol": "NTMT1",
  "gene": "UniProtKB:Q9BV86",
  "gene_name": "N-terminal Xaa-Pro-Lys N-methyltransferase 1",
  "term_id": "GO:0071885"
}